capsorubin synthase activity [GO:0052728] (molecular function) Also known as: CCS, capsanthin-capsorubin synthase activity, ketoxanthophyll synthase activity, violaxanthin-capsorubin isomerase (ketone-forming) activity Relationships: is a type of intramolecular oxidoreductase activity [GO:0016860] Definition: Catalysis of the reaction: all-trans-violaxanthin = all-trans-capsorubin. Sources: RHEA:21752